{
  "gene_symbol": "SLC36A2",
  "term_label": "proline transmembrane transport",
  "gene": "UniProtKB:Q495M3",
  "term_id": "GO:0035524",
  "gene_name": "Proton-coupled amino acid transporter 2"
}